{
  "gene_symbol": "PCDH15",
  "term_id": "GO:0007605",
  "gene": "UniProtKB:Q96QU1",
  "term_label": "sensory perception of sound",
  "gene_name": "Protocadherin-15"
}